{
  "term_id": "GO:0032287",
  "gene_symbol": "PRX",
  "gene_name": "Periaxin",
  "gene": "UniProtKB:Q9BXM0",
  "term_label": "peripheral nervous system myelin maintenance"
}